{
  "term_id": "GO:0035336",
  "term_label": "long-chain fatty-acyl-CoA metabolic process",
  "gene": "UniProtKB:Q96K12",
  "gene_symbol": "FAR2",
  "gene_name": "Fatty acyl-CoA reductase 2"
}